{
  "gene_symbol": "GRPR",
  "term_label": "plasma membrane",
  "gene_name": "Gastrin-releasing peptide receptor",
  "gene": "UniProtKB:P30550",
  "term_id": "GO:0005886"
}